cellular response to copper ion starvation [GO:0035874] (biological process) Definition: Any process that results in a change in state or activity of a cell (in terms of movement, secretion, enzyme production, gene expression, etc.) as a result of deprivation of copper ions. References: PMID:16467469 Sources: GOC:vw Also known as: cellular response to copper starvation Relationships: is a type of GO:0009267; is a type of GO:0120126